{
  "gene_symbol": "CASQ2",
  "term_label": "sarcoplasmic reticulum lumen",
  "gene": "UniProtKB:O14958",
  "gene_name": "Calsequestrin-2",
  "term_id": "GO:0033018"
}